ergothioneine transmembrane transporter activity [GO:0170001] (molecular function) Definition: Enables the transfer of ergothioneine from one side of a membrane to the other. Relationships: is_a transmembrane transporter activity [GO:0022857] References: PMID:15795384, PMID:20601551, PMID:29530864